positive regulation of NAD metabolic process [GO:1902690] (biological process) Subtypes: positive regulation of 'de novo' NAD biosynthetic process from L-tryptophan [GO:1905014] Relationships: is a type of GO:1900544; is a type of GO:1902688; RO_0002213 NAD+ metabolic process [GO:0019674] References: PMID:19846558 Sources: GOC:TermGenie, GOC:di, GO_REF:0000058 Definition: Any process that activates or increases the frequency, rate or extent of NAD metabolic process. Also known as: positive regulation of NAD (oxidized) metabolic process, positive regulation of NAD (oxidized) metabolism, positive regulation of NAD metabolism, positive regulation of nicotinamide adenine dinucleotide metabolic process, positive regulation of nicotinamide adenine dinucleotide metabolism, positive regulation of oxidized NAD metabolic process, positive regulation of oxidized NAD metabolism, positive regulation of oxidized nicotinamide adenine dinucleotide metabolic process, positive regulation of oxidized nicotinamide adenine dinucleotide metabolism, up regulation of NAD (oxidized) metabolic process, up regulation of NAD (oxidized) metabolism, up regulation of NAD metabolic process, up regulation of NAD metabolism, up regulation of nicotinamide adenine dinucleotide metabolic process, up regulation of nicotinamide adenine dinucleotide metabolism, up regulation of oxidized NAD metabolic process, up regulation of oxidized NAD metabolism, up regulation of oxidized nicotinamide adenine dinucleotide metabolic process, up regulation of oxidized nicotinamide adenine dinucleotide metabolism, up-regulation of NAD (oxidized) metabolic process, up-regulation of NAD (oxidized) metabolism, up-regulation of NAD metabolic process, up-regulation of NAD metabolism, up-regulation of nicotinamide adenine dinucleotide metabolic process, up-regulation of nicotinamide adenine dinucleotide metabolism, up-regulation of oxidized NAD metabolic process, up-regulation of oxidized NAD metabolism, up-regulation of oxidized nicotinamide adenine dinucleotide metabolic process, up-regulation of oxidized nicotinamide adenine dinucleotide metabolism, upregulation of NAD (oxidized) metabolic process, upregulation of NAD (oxidized) metabolism, upregulation of NAD metabolic process, upregulation of NAD metabolism, upregulation of nicotinamide adenine dinucleotide metabolic process, upregulation of nicotinamide adenine dinucleotide metabolism, upregulation of oxidized NAD metabolic process, upregulation of oxidized NAD metabolism, upregulation of oxidized nicotinamide adenine dinucleotide metabolic process, upregulation of oxidized nicotinamide adenine dinucleotide metabolism, activation of NAD (oxidized) metabolic process, activation of NAD (oxidized) metabolism, activation of NAD metabolic process, activation of NAD metabolism, activation of NAD phosphorylation and dephosphorylation, activation of nicotinamide adenine dinucleotide metabolic process, activation of nicotinamide adenine dinucleotide metabolism, activation of oxidized NAD metabolic process, activation of oxidized NAD metabolism, activation of oxidized nicotinamide adenine dinucleotide metabolic process, activation of oxidized nicotinamide adenine dinucleotide metabolism, positive regulation of NAD phosphorylation and dephosphorylation, up regulation of NAD phosphorylation and dephosphorylation, up-regulation of NAD phosphorylation and dephosphorylation, upregulation of NAD phosphorylation and dephosphorylation